{
  "gene_symbol": "ZNF347",
  "gene_name": "Zinc finger protein 347",
  "gene": "UniProtKB:Q96SE7",
  "term_label": "DNA-binding transcription factor activity, RNA polymerase II-specific",
  "term_id": "GO:0000981"
}